{
  "term_label": "mRNA 3'-UTR binding",
  "gene_symbol": "PABPC3",
  "gene": "UniProtKB:Q9H361",
  "term_id": "GO:0003730",
  "gene_name": "Polyadenylate-binding protein 3"
}